resveratrol binding [GO:1905594] (molecular function) Relationships: is a type of binding [GO:0005488] Definition: Binding to resveratrol. Note: (5-(aziridin-1-yl)-2,4-dinitrobenzamide References: PMID:18254726 Sources: GOC:TermGenie, GO_REF:0000067